{
  "gene": "UniProtKB:B7ZC32",
  "gene_symbol": "KIF28P",
  "term_id": "GO:0005871",
  "term_label": "kinesin complex",
  "gene_name": "Kinesin-like protein KIF28P"
}